{
  "gene_name": "DNA-directed primase_polymerase protein",
  "gene_symbol": "PRIMPOL",
  "term_label": "nucleus",
  "gene": "UniProtKB:Q96LW4",
  "term_id": "GO:0005634"
}